{
  "gene": "UniProtKB:Q6ZV70",
  "gene_name": "LanC-like protein 3",
  "term_label": "Unknown biological process",
  "gene_symbol": "LANCL3",
  "term_id": "UNKNOWN:0002"
}